{
  "gene_symbol": "OOSP1",
  "gene_name": "Putative oocyte-secreted protein 1 homolog",
  "term_id": "UNKNOWN:0003",
  "term_label": "Unknown cellular component",
  "gene": "UniProtKB:A8MZH6"
}